{
  "gene": "UniProtKB:P0DTL5",
  "term_id": "UNKNOWN:0003",
  "term_label": "Unknown cellular component",
  "gene_symbol": "TMEM276",
  "gene_name": "Transmembrane protein 276"
}